{
  "gene": "UniProtKB:O75954",
  "gene_symbol": "TSPAN9",
  "term_label": "Unknown biological process",
  "term_id": "UNKNOWN:0002",
  "gene_name": "Tetraspanin-9"
}